{
  "gene_name": "Prostaglandin E synthase 3",
  "term_id": "GO:0051131",
  "term_label": "chaperone-mediated protein complex assembly",
  "gene": "UniProtKB:Q15185",
  "gene_symbol": "PTGES3"
}